{
  "gene": "UniProtKB:Q538Z0",
  "gene_symbol": "LUZP6",
  "term_label": "Unknown biological process",
  "gene_name": "Leucine zipper protein 6",
  "term_id": "UNKNOWN:0002"
}